ribosylnicotinamide kinase activity [GO:0050262] (molecular function) References: PMID:17914902 Sources: RHEA:14017 Relationships: is a type of kinase activity [GO:0016301]; is a type of phosphotransferase activity, alcohol group as acceptor [GO:0016773] Also known as: nicotinamide riboside kinase activity, ATP:N-ribosylnicotinamide 5'-phosphotransferase activity, ribosylnicotinamide kinase (phosphorylating) Definition: Catalysis of the reaction: beta-nicotinamide D-riboside + ATP = beta-nicotinamide D-ribonucleotide + ADP + H+.